{
  "term_label": "chromatin binding",
  "gene_symbol": "LRWD1",
  "term_id": "GO:0003682",
  "gene_name": "Leucine-rich repeat and WD repeat-containing protein 1",
  "gene": "UniProtKB:Q9UFC0"
}